{
  "gene_name": "7-alpha-hydroxycholest-4-en-3-one 12-alpha-hydroxylase",
  "gene_symbol": "CYP8B1",
  "term_id": "UNKNOWN:0002",
  "gene": "UniProtKB:Q9UNU6",
  "term_label": "Unknown biological process"
}